{
  "gene_symbol": "MAF1",
  "gene": "UniProtKB:Q9H063",
  "gene_name": "Repressor of RNA polymerase III transcription MAF1 homolog",
  "term_label": "nucleus",
  "term_id": "GO:0005634"
}